{
  "gene": "UniProtKB:Q96RU7",
  "gene_name": "Tribbles homolog 3",
  "term_label": "mitogen-activated protein kinase kinase binding",
  "gene_symbol": "TRIB3",
  "term_id": "GO:0031434"
}